{
  "term_label": "Unknown molecular function",
  "gene": "UniProtKB:Q5T5N4",
  "term_id": "UNKNOWN:0001",
  "gene_name": "Uncharacterized protein C6orf118",
  "gene_symbol": "C6orf118"
}